regulation of T-helper 17 type immune response [GO:2000316] (biological process) Definition: Any process that modulates the frequency, rate or extent of T-helper 17 type immune response. Subtypes: negative regulation of T-helper 17 type immune response [GO:2000317], positive regulation of T-helper 17 type immune response [GO:2000318], regulation of T-helper 17 cell differentiation [GO:2000319] Sources: GOC:BHF, GOC:mah Relationships: is a type of GO:0002822; regulates T-helper 17 type immune response [GO:0072538] Also known as: regulation of Th17 immune response